{
  "gene_symbol": "RPL9P9",
  "gene_name": "Large ribosomal subunit protein uL6",
  "gene": "UniProtKB:P32969",
  "term_label": "cytosolic large ribosomal subunit",
  "term_id": "GO:0022625"
}